ricinine nitrilase activity [GO:0047426] (molecular function) Definition: Catalysis of the reaction: H2O + ricinine = NH3 + 3-carboxy-4-methoxy-N-methyl-2-pyridone. Sources: EC:3.5.5.2 Relationships: is a type of nitrilase activity [GO:0000257] Also known as: ricinine aminohydrolase activity